{
  "gene_symbol": "AQP2",
  "term_label": "plasma membrane",
  "gene_name": "Aquaporin-2",
  "gene": "UniProtKB:P41181",
  "term_id": "GO:0005886"
}